gamma-aminobutyric acid:proton antiporter activity [GO:0140800] (molecular function) Definition: Enables the transfer of a solute or solutes from one side of a membrane to the other according to the reaction: 4-aminobutanoate(out) + H+(in) = 4-aminobutanoate(in) + H+(out). References: PMID:16701208, PMID:26912364, PMID:27601664 Relationships: is a type of proton transmembrane transporter activity [GO:0015078]; is a type of gamma-aminobutyric acid transmembrane transporter activity [GO:0015185]; is a type of secondary active monocarboxylate transmembrane transporter activity [GO:0015355]; is a type of amino acid:monoatomic cation antiporter activity [GO:0140848]